{
  "gene_symbol": "MICB",
  "gene_name": "MHC class I polypeptide-related sequence B",
  "term_id": "UNKNOWN:0001",
  "term_label": "Unknown molecular function",
  "gene": "UniProtKB:Q29980"
}